hydroxymandelonitrile lyase activity [GO:0050419] (molecular function) Also known as: hydroxynitrile lyase activity, (S)-4-hydroxymandelonitrile 4-hydroxybenzaldehyde-lyase (cyanide-forming), (S)-4-hydroxymandelonitrile hydroxybenzaldehyde-lyase activity, sorghum hydroxynitrile lyase activity Sources: RHEA:15977 Relationships: is a type of aldehyde-lyase activity [GO:0016832] Definition: Catalysis of the reaction: 4-hydroxymandelonitrile = 4-hydroxybenzaldehyde + hydrocyanate.